{
  "term_id": "UNKNOWN:0001",
  "gene_symbol": "FAM174C",
  "gene_name": "Protein FAM174C",
  "term_label": "Unknown molecular function",
  "gene": "UniProtKB:Q9BVV8"
}